{
  "term_id": "GO:0090307",
  "gene": "UniProtKB:O75122",
  "gene_symbol": "CLASP2",
  "term_label": "mitotic spindle assembly",
  "gene_name": "CLIP-associating protein 2"
}